{
  "term_id": "GO:0004930",
  "gene": "UniProtKB:Q7RTX1",
  "gene_name": "Taste receptor type 1 member 1",
  "gene_symbol": "TAS1R1",
  "term_label": "G protein-coupled receptor activity"
}